{
  "term_id": "GO:0005634",
  "gene": "UniProtKB:Q9H9J4",
  "term_label": "nucleus",
  "gene_symbol": "USP42",
  "gene_name": "Ubiquitin carboxyl-terminal hydrolase 42"
}